{
  "gene": "UniProtKB:Q9HD47",
  "term_label": "regulation of membrane depolarization during cardiac muscle cell action potential",
  "gene_name": "Ran guanine nucleotide release factor",
  "gene_symbol": "RANGRF",
  "term_id": "GO:1900825"
}